{
  "gene": "UniProtKB:Q9H9V9",
  "gene_name": "2-oxoglutarate and iron-dependent oxygenase JMJD4",
  "gene_symbol": "JMJD4",
  "term_label": "sequence-specific DNA binding",
  "term_id": "GO:0043565"
}